butyryl-CoA catabolic process to butyrate [GO:0044581] (biological process) Regulation: regulated by regulation of butyryl-CoA catabolic process to butyrate [GO:1900500]; negatively regulated by negative regulation of butyryl-CoA catabolic process to butyrate [GO:1900501]; RO_0002213 by positive regulation of butyryl-CoA catabolic process to butyrate [GO:1900502] Also known as: butyryl-CoA catabolism to butyrate Definition: The chemical reactions a resulting in the resulting in the breakdown of butyryl-CoA to form butyrate. References: PMID:19539744 Sources: GOC:mengo_curators, GOC:tt Relationships: is a type of butyryl-CoA catabolic process [GO:0044580]; is a type of butyrate biosynthetic process [GO:0046358]